imaginal disc fusion, thorax closure [GO:0046529] (biological process) Sources: http://sdb.bio.purdue.edu/fly/gene/fos4.htm Definition: The joining of the parts of the wing imaginal discs, giving rise to the adult thorax. Relationships: is_a post-embryonic animal morphogenesis [GO:0009886]; is part of imaginal disc fusion [GO:0046528]